{
  "gene_name": "Ubiquitin-conjugating enzyme E2 variant 3",
  "gene_symbol": "UEVLD",
  "term_label": "endosome to lysosome transport",
  "gene": "UniProtKB:Q8IX04",
  "term_id": "GO:0008333"
}